{
  "gene_symbol": "CEACAM4",
  "gene": "UniProtKB:O75871",
  "term_label": "plasma membrane",
  "gene_name": "Carcinoembryonic antigen-related cell adhesion molecule 4",
  "term_id": "GO:0005886"
}